{
  "term_label": "outer dense fiber",
  "term_id": "GO:0001520",
  "gene_name": "Transmembrane protein 232",
  "gene": "UniProtKB:C9JQI7",
  "gene_symbol": "TMEM232"
}